{
  "gene": "UniProtKB:O95573",
  "gene_symbol": "ACSL3",
  "term_label": "neuron differentiation",
  "term_id": "GO:0030182",
  "gene_name": "Fatty acid CoA ligase Acsl3"
}